{
  "gene": "UniProtKB:Q9BWD3",
  "gene_name": "Retrotransposon Gag-like protein 8A",
  "gene_symbol": "RTL8A",
  "term_label": "Unknown biological process",
  "term_id": "UNKNOWN:0002"
}